menopause [GO:0042697] (biological process) Definition: Cessation of menstruation, occurring in (e.g.) the human female usually around the age of 50. References: PMID:18495681 Sources: GOC:curators Note: Note that this term should not be used for direct annotation. If you are trying to make an annotation to x phase, it is likely that the correct annotation is 'regulation of x/y phase transition' or to a process which occurs during the reported phase. To capture the phase when a specific location or process is observed, the phase term can be used in an annotation extension (PMID:24885854) applied to a cellular component term (with the relation exists_during) or a biological process term (with the relation happens_during). Relationships: is a type of menstrual cycle phase [GO:0022601]; is a type of reproductive senescence [GO:1990636]